{
  "term_id": "UNKNOWN:0003",
  "term_label": "Unknown cellular component",
  "gene_symbol": "TRAJ48",
  "gene_name": "T cell receptor alpha joining 48 (Fragment)",
  "gene": "UniProtKB:A0A075B6V3"
}